{
  "gene_symbol": "KLHL38",
  "term_label": "Cul3-RING ubiquitin ligase complex",
  "gene_name": "Kelch-like protein 38",
  "gene": "UniProtKB:Q2WGJ6",
  "term_id": "GO:0031463"
}